G protein-coupled receptor catabolic process [GO:1990172] (biological process) Relationships: is a type of receptor catabolic process [GO:0032801]; is a type of negative regulation of G protein-coupled receptor signaling pathway [GO:0045744] References: PMID:12142540, PMID:23954414 Definition: The chemical reactions and pathways resulting in the breakdown of a G protein-coupled receptor. Also known as: G-protein coupled receptor catabolic process